{
  "term_id": "UNKNOWN:0001",
  "gene": "UniProtKB:O00220",
  "gene_name": "Tumor necrosis factor receptor superfamily member 10A",
  "term_label": "Unknown molecular function",
  "gene_symbol": "TNFRSF10A"
}